{
  "gene_name": "E3 ubiquitin-protein ligase UBR3",
  "term_id": "GO:0071596",
  "term_label": "ubiquitin-dependent protein catabolic process via the N-end rule pathway",
  "gene": "UniProtKB:Q6ZT12",
  "gene_symbol": "UBR3"
}